selenocystathionine gamma-lyase activity [GO:0098606] (MF) References: PMID:6456763 Sources: RHEA:31151 Definition: Catalysis of the reaction:L-selenocystathionine + H2O = L-selenocysteine + 2-oxobutanoate + NH4+. Relationships: is a type of GO:0016846